{
  "gene": "UniProtKB:Q99611",
  "gene_symbol": "SEPHS2",
  "term_label": "selenocysteine biosynthetic process",
  "term_id": "GO:0016260",
  "gene_name": "Selenide, water dikinase 2"
}